{
  "gene_name": "Tachykinin-4",
  "term_label": "tachykinin receptor signaling pathway",
  "gene_symbol": "TAC4",
  "term_id": "GO:0007217",
  "gene": "UniProtKB:Q86UU9"
}